{
  "gene": "UniProtKB:Q2T9L4",
  "term_id": "GO:0060080",
  "gene_symbol": "INSYN1",
  "term_label": "inhibitory postsynaptic potential",
  "gene_name": "Inhibitory synaptic factor 1"
}